{
  "term_label": "endoplasmic reticulum exit site",
  "term_id": "GO:0070971",
  "gene_name": "Protein transport protein Sec23B",
  "gene_symbol": "SEC23B",
  "gene": "UniProtKB:Q15437"
}